protein kinase CK2 complex [GO:0005956] (cellular component) Relationships: is a type of intracellular protein-containing complex [GO:0140535]; is a type of serine/threonine protein kinase complex [GO:1902554] Definition: A protein complex that possesses protein serine/threonine kinase activity, and contains two catalytic alpha subunits and two regulatory beta subunits. Protein kinase CK2 complexes are found in nearly every subcellular compartment, and can phosphorylate many protein substrates in addition to casein. Note: Note that this term represents a location and not a function; the activity possessed by this complex is mentioned in the definition for the purpose of describing and distinguishing the complex. Also known as: casein kinase II complex References: PMID:10994779 Sources: GOC:mah